sperm DNA condensation [GO:0035092] (biological process) References: PMID:11735001 Sources: GOC:bf Relationships: is a type of chromatin organization [GO:0006325]; is part of GO:0007289 Also known as: sperm chromatin condensation, spermatogenesis, exchange of chromosomal proteins Definition: The progressive compaction of the spermatid chromatin so that it reaches a level of condensation that is not compatible with nuclear activities such as transcription or DNA replication.